{
  "gene": "UniProtKB:P18206",
  "gene_name": "Vinculin",
  "term_label": "cell adhesion",
  "gene_symbol": "VCL",
  "term_id": "GO:0007155"
}